{
  "term_id": "GO:0007030",
  "gene": "UniProtKB:A6NCC3",
  "gene_name": "Golgin subfamily A member 8O",
  "gene_symbol": "GOLGA8O",
  "term_label": "Golgi organization"
}